{
  "gene": "UniProtKB:Q7Z2G1",
  "gene_name": "Histone H2B type W-T",
  "term_label": "DNA binding",
  "gene_symbol": "H2BW1",
  "term_id": "GO:0003677"
}